{
  "gene_symbol": "ARGFX",
  "term_id": "GO:0005634",
  "gene_name": "Arginine-fifty homeobox",
  "gene": "UniProtKB:A6NJG6",
  "term_label": "nucleus"
}